disulfoglucosamine-6-sulfatase activity [GO:0047871] (molecular function) Relationships: is a type of sulfuric ester hydrolase activity [GO:0008484] Sources: EC:3.1.6.11, RHEA:15517 Definition: Catalysis of the reaction: N(2),6-disulfo-D-glucosamine + H2O = N-sulfo-D-glucosamine + H+ + sulfate. Also known as: disulphoglucosamine-6-sulphatase activity, 6,N-disulfoglucosamine 6-O-sulfohydrolase activity, N,6-O-disulfo-D-glucosamine 6-sulfohydrolase activity, N-sulfoglucosamine-6-sulfatase activity